{
  "gene_name": "Ras-related protein Rab-5C",
  "gene_symbol": "RAB5C",
  "term_id": "GO:0012505",
  "term_label": "endomembrane system",
  "gene": "UniProtKB:P51148"
}